{
  "term_label": "odorant binding",
  "gene_name": "Olfactory receptor 10T2",
  "term_id": "GO:0005549",
  "gene_symbol": "OR10T2",
  "gene": "UniProtKB:Q8NGX3"
}